acquisition of mycelium reproductive competence [GO:0097737] (biological process) Definition: A maturation process by which an organism acquires the ability to reproduce. In fungi, reproductive competence only occurs in a population of filamentous cells that form a mycelium. References: PMID:23864594 Sources: GOC:di Relationships: is a type of GO:0032502 Also known as: mycelium developmental competence